{
  "gene_name": "Cholesterol side-chain cleavage enzyme, mitochondrial",
  "gene": "UniProtKB:P05108",
  "term_label": "cortisol metabolic process",
  "gene_symbol": "CYP11A1",
  "term_id": "GO:0034650"
}